chromosome [GO:0005694] (cellular component) Relationships: is a type of intracellular membraneless organelle [GO:0043232] Also known as: interphase chromosome, prophase chromosome, chromatid Subtypes: nuclear chromosome [GO:0000228], mitochondrial chromosome [GO:0000262], condensed chromosome [GO:0000793], sex chromosome [GO:0000803], polytene chromosome [GO:0005700], plastid chromosome [GO:0009508], autosome [GO:0030849] Note: Chromosomes include parts that are not part of the chromatin. Examples include the kinetochore. Definition: A structure composed of a very long molecule of DNA and associated proteins (e.g. histones) that carries hereditary information. Sources: ISBN:0198547684